{
  "term_label": "mitotic cell cycle",
  "gene": "UniProtKB:Q9UGJ1",
  "gene_symbol": "TUBGCP4",
  "term_id": "GO:0000278",
  "gene_name": "Gamma-tubulin complex component 4"
}